galactomannan metabolic process [GO:0051069] (biological process) Relationships: is a type of substituted mannan metabolic process [GO:0006080] Also known as: galactomannan metabolism References: PMID:30701316, PMID:33012173 Definition: The chemical reactions and pathways involving galactomannan, a polysaccharide composed of D-galactose and D-mannose. The mannose units form the backbone structure (a linear main chain) with the D-galactose as single side units. Subtypes: galactomannan biosynthetic process [GO:0051070], GO:0051682